{
  "term_label": "Unknown cellular component",
  "gene_symbol": "A0A8I5KXM2",
  "term_id": "UNKNOWN:0003",
  "gene_name": "Uncharacterized protein",
  "gene": "UniProtKB:A0A8I5KXM2"
}